{
  "gene_symbol": "ARRB2",
  "gene_name": "Beta-arrestin-2",
  "term_id": "GO:0005737",
  "gene": "UniProtKB:P32121",
  "term_label": "cytoplasm"
}